{
  "term_id": "GO:0003365",
  "gene_name": "Angiomotin-like protein 2",
  "term_label": "establishment of cell polarity involved in ameboidal cell migration",
  "gene": "UniProtKB:Q9Y2J4",
  "gene_symbol": "AMOTL2"
}